specification of petal number [GO:0048834] (biological process) Relationships: is a type of specification of floral organ number [GO:0048833]; is part of GO:0048465 Sources: GOC:tb Definition: Any process that modulates the number of petals formed in a flower.